{
  "gene_symbol": "BCL2L13",
  "term_label": "Unknown molecular function",
  "gene": "UniProtKB:Q9BXK5",
  "term_id": "UNKNOWN:0001",
  "gene_name": "Bcl-2-like protein 13"
}